circadian mating behavior [GO:0035648] (BP) Also known as: circadian mating behaviour, circadian mating rhythm References: PMID:11470898, PMID:17276917 Sources: GOC:bf, GOC:dos Definition: The fluctuation in mating behavior that occurs over an approximately 24 hour cycle. Relationships: is a type of GO:0007617; is a type of circadian behavior [GO:0048512]